{
  "term_label": "cytokine activity",
  "gene": "UniProtKB:P01563",
  "gene_symbol": "IFNA2",
  "term_id": "GO:0005125",
  "gene_name": "Interferon alpha-2"
}